{
  "gene_symbol": "CDC42EP2",
  "gene": "UniProtKB:O14613",
  "term_id": "GO:0005856",
  "term_label": "cytoskeleton",
  "gene_name": "Cdc42 effector protein 2"
}